nucleoside diphosphate biosynthetic process [GO:0009133] (biological process) Also known as: nucleoside diphosphate anabolism, nucleoside diphosphate biosynthesis, nucleoside diphosphate formation, nucleoside diphosphate synthesis Definition: The chemical reactions and pathways resulting in the formation of a nucleoside diphosphate, a compound consisting of a nucleobase linked to a deoxyribose or ribose sugar esterified with diphosphate on the sugar. Relationships: is_a nucleoside diphosphate metabolic process [GO:0009132]; is a type of nucleoside phosphate biosynthetic process [GO:1901293] Sources: GOC:go_curators, ISBN:0198506732 Subtypes: purine nucleoside diphosphate biosynthetic process [GO:0009136], GO:0009139, ribonucleoside diphosphate biosynthetic process [GO:0009188], deoxyribonucleoside diphosphate biosynthetic process [GO:0009189]